{
  "gene_symbol": "CFAP206",
  "term_label": "axoneme",
  "term_id": "GO:0005930",
  "gene": "UniProtKB:Q8IYR0",
  "gene_name": "Cilia- and flagella-associated protein 206"
}